pro-T cell differentiation [GO:0002572] (biological process) Definition: The process in which a precursor cell type acquires the specialized features of a pro-T cell. Pro-T cells are the earliest stage of the T cell lineage but are not fully committed. Relationships: is a type of lymphoid progenitor cell differentiation [GO:0002320]; BFO_0000050 GO:0030217 Also known as: pro-T lymphocyte differentiation Regulation: regulated by GO:2000174; negatively regulated by negative regulation of pro-T cell differentiation [GO:2000175]; positively regulated by positive regulation of pro-T cell differentiation [GO:2000176] Sources: GOC:add, ISBN:0781735149